{
  "gene_symbol": "CHRFAM7A",
  "term_label": "plasma membrane",
  "term_id": "GO:0005886",
  "gene": "UniProtKB:Q494W8",
  "gene_name": "CHRNA7-FAM7A fusion protein"
}